{
  "gene_symbol": "CTDSP2",
  "gene": "UniProtKB:O14595",
  "term_id": "UNKNOWN:0002",
  "gene_name": "Carboxy-terminal domain RNA polymerase II polypeptide A small phosphatase 2",
  "term_label": "Unknown biological process"
}